{
  "gene_symbol": "DPY19L4",
  "term_id": "UNKNOWN:0002",
  "gene": "UniProtKB:Q7Z388",
  "gene_name": "Probable C-mannosyltransferase DPY19L4",
  "term_label": "Unknown biological process"
}